{
  "gene_symbol": "PRKDC",
  "gene": "UniProtKB:P78527",
  "term_label": "double-strand break repair",
  "term_id": "GO:0006302",
  "gene_name": "DNA-dependent protein kinase catalytic subunit"
}